interferon-mediated signaling pathway [GO:0140888] (biological process) Relationships: is a type of cytokine-mediated signaling pathway [GO:0019221] Subtypes: GO:0038196, type II interferon-mediated signaling pathway [GO:0060333], type I interferon-mediated signaling pathway [GO:0060337] Definition: The series of molecular signals initiated by type II interferon binding to its receptor on the surface of a target cell, and ending with the regulation of a downstream cellular process, e.g. transcription. Type II interferon is also known as interferon-gamma. References: PMID:32464097 Sources: GOC:add, GOC:dph, GOC:signaling Also known as: interferon signaling pathway, interferon-activated signaling pathway